{
  "term_id": "UNKNOWN:0003",
  "gene_symbol": "SMPD4",
  "gene_name": "Sphingomyelin phosphodiesterase 4",
  "gene": "UniProtKB:Q9NXE4",
  "term_label": "Unknown cellular component"
}